{
  "term_id": "GO:0004869",
  "gene_name": "Putative pituitary tumor-transforming gene 3 protein",
  "term_label": "cysteine-type endopeptidase inhibitor activity",
  "gene_symbol": "PTTG3P",
  "gene": "UniProtKB:Q9NZH4"
}